O-antigen ligase activity [GO:0008754] (molecular function) Definition: Catalysis of the reaction: a lipid-linked O antigen + a lipid A-core oligosaccharide = a lipopolysaccharide + a polyisoprenyl diphosphate. Sources: EC:2.4.99.26 Relationships: is a type of glycosyltransferase activity [GO:0016757]